{
  "gene_name": "Ectoderm-neural cortex protein 1",
  "gene_symbol": "ENC1",
  "term_id": "GO:1990756",
  "term_label": "ubiquitin-like ligase-substrate adaptor activity",
  "gene": "UniProtKB:O14682"
}